nephrocyte filtration [GO:0097206] (biological process) Definition: The process by which hemolymph is filtered based on size and charge through a nephrocyte filtration barrier formed by the basement membrane and nephrocyte diaphragm. References: PMID:18971929 Sources: GOC:sart Relationships: is a type of renal filtration [GO:0097205]